{
  "gene_symbol": "GJC2",
  "term_id": "GO:0007267",
  "gene_name": "Gap junction gamma-2 protein",
  "term_label": "cell-cell signaling",
  "gene": "UniProtKB:Q5T442"
}